{
  "gene_symbol": "MYO1B",
  "gene_name": "Unconventional myosin-Ib",
  "gene": "UniProtKB:O43795",
  "term_label": "brush border",
  "term_id": "GO:0005903"
}